inositol-1,3,4-trisphosphate 1-phosphatase activity [GO:0052829] (molecular function) Definition: Catalysis of the reaction: D-myo-inositol 1,3,4-trisphosphate + H2O = myo-inositol 3,4-bisphosphate + phosphate. Relationships: is a type of GO:0046030 Sources: GOC:ai